{
  "gene": "UniProtKB:Q16526",
  "gene_symbol": "CRY1",
  "gene_name": "Cryptochrome-1",
  "term_label": "cytoplasm",
  "term_id": "GO:0005737"
}